{
  "term_label": "signaling adaptor activity",
  "term_id": "GO:0035591",
  "gene_name": "Signal-transducing adaptor protein 1",
  "gene": "UniProtKB:Q9ULZ2",
  "gene_symbol": "STAP1"
}